COPI vesicle coat [GO:0030126] (cellular component) Also known as: coatomer Definition: One of two multimeric complexes that forms a membrane vesicle coat. The mammalian COPI subunits are called alpha-, beta-, beta'-, gamma-, delta-, epsilon- and zeta-COP. Vesicles with COPI coats are found associated with Golgi membranes at steady state. References: PMID:11252894 Sources: GOC:mah Relationships: is a type of GO:0030120; is part of Golgi apparatus [GO:0005794]; is part of COPI-coated vesicle membrane [GO:0030663]